{
  "gene_symbol": "MSH2",
  "term_label": "mitotic recombination",
  "gene": "UniProtKB:P43246",
  "gene_name": "DNA mismatch repair protein Msh2",
  "term_id": "GO:0006312"
}